{
  "term_id": "GO:0007186",
  "gene_symbol": "TAAR5",
  "term_label": "G protein-coupled receptor signaling pathway",
  "gene_name": "Trace amine-associated receptor 5",
  "gene": "UniProtKB:O14804"
}